negative regulation of interleukin-2 production [GO:0032703] (biological process) Also known as: down regulation of interleukin-2 production, down-regulation of interleukin-2 production, downregulation of interleukin-2 production, negative regulation of IL-2 production, inhibition of interleukin-2 production, negative regulation of interleukin-2 biosynthetic process, negative regulation of interleukin-2 secretion Definition: Any process that stops, prevents, or reduces the frequency, rate, or extent of interleukin-2 production. Sources: GOC:mah Relationships: is a type of GO:0001818; is a type of regulation of interleukin-2 production [GO:0032663]; negatively regulates interleukin-2 production [GO:0032623]